{
  "term_id": "UNKNOWN:0001",
  "gene": "UniProtKB:Q674X7",
  "term_label": "Unknown molecular function",
  "gene_symbol": "KAZN",
  "gene_name": "Kazrin"
}